{
  "gene_name": "Nicotinate phosphoribosyltransferase",
  "gene_symbol": "NAPRT",
  "gene": "UniProtKB:Q6XQN6",
  "term_label": "nicotinate phosphoribosyltransferase activity",
  "term_id": "GO:0004516"
}